mitochondrial glycyl-tRNA aminoacylation [GO:0070150] (BP) Definition: The process of coupling glycine to glycyl-tRNA in a mitochondrion, catalyzed by glycyl-tRNA synthetase. In tRNA aminoacylation, the amino acid is first activated by linkage to AMP and then transferred to either the 2'- or the 3'-hydroxyl group of the 3'-adenosine residue of the tRNA. Relationships: is a type of glycyl-tRNA aminoacylation [GO:0006426]; is a type of tRNA aminoacylation for mitochondrial protein translation [GO:0070127] Sources: GOC:mah, GOC:mcc